propionyl-CoA biosynthetic process [GO:1902860] (biological process) Also known as: propionyl-CoA anabolism, propionyl-CoA biosynthesis, propionyl-CoA formation, propionyl-CoA synthesis Relationships: is_a GO:0046949; is a type of GO:1902858 Definition: The chemical reactions and pathways resulting in the formation of propionyl-CoA. References: PMID:15514053 Sources: GOC:TermGenie, GOC:mengo_curators, GO_REF:0000068